establishment of RNA localization [GO:0051236] (biological process) Definition: The directed movement of RNA to a specific location. Sources: GOC:ai Subtypes: establishment of pole plasm mRNA localization [GO:0046595], RNA transport [GO:0050658], establishment of RNA localization to telomere [GO:0097694] Also known as: RNA positioning, RNA recruitment, establishment of RNA localisation Relationships: is a type of establishment of localization [GO:0051234]; is part of RNA localization [GO:0006403]